cellular response to nitrogen compound [GO:1901699] (biological process) Definition: Any process that results in a change in state or activity of a cell (in terms of movement, secretion, enzyme production, gene expression, etc.) as a result of a nitrogen compound stimulus. Sources: GOC:TermGenie, GOC:pr Also known as: cellular response to nitrogen molecular entity Note: Note that this term is in the subset of terms that should not be used for direct gene product annotation. Instead, select a child term or, if no appropriate child term exists, please request a new term. Direct annotations to this term may be amended during annotation QC. Relationships: is a type of cellular response to chemical stimulus [GO:0070887]; is a type of GO:1901698 Subtypes: cellular response to nitrogen dioxide [GO:0035714], cellular response to trichostatin A [GO:0035984], GO:0036280, cellular response to L-cysteine [GO:0036346], cellular response to methionine [GO:0061431], cellular response to 1-aminocyclopropane-1-carboxylic acid [GO:0071213], cellular response to peptidoglycan [GO:0071224], GO:0071225, cellular response to folic acid [GO:0071231], cellular response to histidine [GO:0071232], GO:0071233, cellular response to phenylalanine [GO:0071234], cellular response to proline [GO:0071235], cellular response to bacteriocin [GO:0071237], cellular response to ammonium ion [GO:0071242], cellular response to biotin [GO:0071296], GO:0071297, cellular response to vitamin B1 [GO:0071301], cellular response to vitamin B2 [GO:0071302], GO:0071304, cellular response to alkaloid [GO:0071312], cellular response to ATP [GO:0071318], cellular response to cAMP [GO:0071320], GO:0071321, GO:0071323, cellular response to dsRNA [GO:0071359], cellular response to indolebutyric acid stimulus [GO:0071366], cellular response to peptide hormone stimulus [GO:0071375], cellular response to cycloheximide [GO:0071409], cellular response to methotrexate [GO:0071414], cellular response to amine stimulus [GO:0071418], GO:0071420, cellular response to heparin [GO:0071504], cellular response to indole-3-methanol [GO:0071681], cellular response to monoamine stimulus [GO:0071868], cellular response to hydroxyurea [GO:0072711], cellular response to thiabendazole [GO:0072713], cellular response to actinomycin D [GO:0072717], cellular response to amitrole [GO:0072723], cellular response to 4-nitroquinoline N-oxide [GO:0072725], cellular response to diamide [GO:0072738], GO:0072745, cellular response to chloramphenicol [GO:0072747], GO:0072748, GO:0072749, cellular response to L-thialysine [GO:0072751], GO:0072752, cellular response to glutathione [GO:0072753], cellular response to purvalanol A [GO:0072754], cellular response to azide [GO:0097185], cellular response to reactive nitrogen species [GO:1902170], GO:1902350, cellular response to L-arginine [GO:1903577], cellular response to acrylamide [GO:1903938], cellular response to micafungin [GO:1903968], GO:1904102, GO:1904308, GO:1904310, cellular response to 2-O-acetyl-1-O-hexadecyl-sn-glycero-3-phosphocholine [GO:1904317], GO:1904374, cellular response to L-phenylalanine derivative [GO:1904387], cellular response to ciliary neurotrophic factor [GO:1904392], GO:1904403, cellular response to tetrahydrofolate [GO:1904482], cellular response to diphenidol [GO:1904561], GO:1904584, cellular response to putrescine [GO:1904586], cellular response to glycoprotein [GO:1904588], cellular response to dinitrophenol [GO:1904642], cellular response to amyloid-beta [GO:1904646], cellular response to nitroglycerin [GO:1904843], cellular response to L-glutamine [GO:1904845], cellular response to bleomycin [GO:1904976], cellular response to haloperidol [GO:1905120], GO:1905145, cellular response to L-glutamate [GO:1905232], cellular response to cyclosporin A [GO:1905238], cellular response to 3,3',5-triiodo-L-thyronine [GO:1905243], cellular response to miconazole [GO:1905308], GO:1905375, cellular response to glycine [GO:1905430], cellular response to chondroitin 6'-sulfate [GO:1905440], cellular response to chondroitin 4'-sulfate [GO:1905442], cellular response to puromycin [GO:1905795], GO:1905835, cellular response to dsDNA [GO:1990786]